{
  "gene": "UniProtKB:B1ANS9",
  "gene_name": "WD repeat-containing protein 64",
  "gene_symbol": "WDR64",
  "term_label": "Unknown cellular component",
  "term_id": "UNKNOWN:0003"
}